{
  "term_id": "GO:0070985",
  "gene": "UniProtKB:P50613",
  "gene_symbol": "CDK7",
  "gene_name": "Cyclin-dependent kinase 7",
  "term_label": "transcription factor TFIIK complex"
}